cardiac cell fate commitment [GO:0060911] (biological process) Definition: The commitment of cells to specific cardiac cell fates and their capacity to differentiate into cardiac cells. Cardiac cells are cells that comprise the organ which pumps blood through the circulatory system. Relationships: is a type of cell fate commitment [GO:0045165]; is part of cardiocyte differentiation [GO:0035051] Also known as: cardiocyte cell fate commitment Sources: GOC:mtg_heart Subtypes: dorsal vessel aortic cell fate commitment [GO:0035052], GO:0035053, GO:0042684, cardiac muscle cell fate commitment [GO:0060923], His-Purkinje system cell fate commitment [GO:0060934], cardiac fibroblast cell fate commitment [GO:0060937], GO:0060949, cardiac glial cell fate commitment [GO:0060953], endocardial cell fate commitment [GO:0060957], cardiac neuron fate commitment [GO:0060960]